{
  "gene_symbol": "ZNF546",
  "term_id": "GO:0006357",
  "gene": "UniProtKB:Q86UE3",
  "gene_name": "Zinc finger protein 546",
  "term_label": "regulation of transcription by RNA polymerase II"
}